{
  "term_id": "GO:0004713",
  "gene_name": "Homeodomain-interacting protein kinase 3",
  "gene_symbol": "HIPK3",
  "gene": "UniProtKB:Q9H422",
  "term_label": "protein tyrosine kinase activity"
}